{
  "gene_name": "PCI domain-containing protein 2",
  "gene": "UniProtKB:Q5JVF3",
  "gene_symbol": "PCID2",
  "term_id": "GO:0003690",
  "term_label": "double-stranded DNA binding"
}